{
  "term_label": "actin cytoskeleton organization",
  "gene_name": "Alpha-actinin-2",
  "gene_symbol": "ACTN2",
  "term_id": "GO:0030036",
  "gene": "UniProtKB:P35609"
}